{
  "term_label": "endoplasmic reticulum",
  "gene_symbol": "TMF1",
  "gene_name": "TATA element modulatory factor",
  "term_id": "GO:0005783",
  "gene": "UniProtKB:P82094"
}